{
  "term_id": "GO:0034703",
  "term_label": "cation channel complex",
  "gene_symbol": "TRPC5",
  "gene": "UniProtKB:Q9UL62",
  "gene_name": "Short transient receptor potential channel 5"
}